establishment of protein-containing complex localization to telomere [GO:0097695] (biological process) References: PMID:26586433 Sources: GOC:BHF, GOC:BHF_telomere, GOC:rph Also known as: establishment of macromolecular complex localisation to telomere, establishment of macromolecular complex localization to telomere Relationships: is a type of establishment of localization [GO:0051234]; is part of macromolecule localization [GO:0033036] Definition: The directed movement of a protein-containing macromolecular complex to a specific location in the telomeric region of a chromosome. Regulation: regulated by regulation of establishment of protein-containing complex localization to telomere [GO:1904913]; negatively regulated by negative regulation of establishment of protein-containing complex localization to telomere [GO:1904914]; positively regulated by GO:1904915